glycerolipid metabolic process [GO:0046486] (biological process) References: PMID:8906569 Sources: GOC:ai Relationships: is a type of GO:0006629 Subtypes: acylglycerol metabolic process [GO:0006639], glycerophospholipid metabolic process [GO:0006650], glycerolipid biosynthetic process [GO:0045017], GO:0046503 Also known as: glycerolipid metabolism Definition: The chemical reactions and pathways involving glycerolipids, any lipid with a glycerol backbone. Diacylglycerol and phosphatidate are key lipid intermediates of glycerolipid biosynthesis.